{
  "term_label": "Unknown cellular component",
  "gene": "UniProtKB:O95760",
  "term_id": "UNKNOWN:0003",
  "gene_name": "Interleukin-33",
  "gene_symbol": "IL33"
}